{
  "gene": "UniProtKB:Q9Y3Q0",
  "term_id": "UNKNOWN:0002",
  "term_label": "Unknown biological process",
  "gene_symbol": "NAALAD2",
  "gene_name": "N-acetylated-alpha-linked acidic dipeptidase 2"
}